{
  "gene_symbol": "RAB6C",
  "gene_name": "Ras-related protein Rab-6C",
  "term_id": "GO:0006891",
  "gene": "UniProtKB:Q9H0N0",
  "term_label": "intra-Golgi vesicle-mediated transport"
}